{
  "gene_name": "Zinc finger protein 283",
  "term_label": "DNA-binding transcription factor activity, RNA polymerase II-specific",
  "term_id": "GO:0000981",
  "gene_symbol": "ZNF283",
  "gene": "UniProtKB:Q8N7M2"
}